homologous chromosome orientation in meiotic metaphase I [GO:0031619] (biological process) Relationships: is a type of chromosome localization [GO:0050000]; is part of GO:0043060 References: PMID:15062096 Definition: The cell cycle process in which the sister centromeres and kinetochores of one chromosome are fused and orientated so the chromosomes attach to microtubules that emanate from the same spindle pole. This process ensures that homologous l chromosomes are segregated at anaphase of meiosis I. Also known as: homologous chromosome orientation during meiosis, homologous chromosome orientation during meiosis I